{
  "term_label": "ER retention sequence binding",
  "gene_name": "ER lumen protein-retaining receptor 3",
  "term_id": "GO:0046923",
  "gene_symbol": "KDELR3",
  "gene": "UniProtKB:O43731"
}